{
  "term_id": "GO:0005737",
  "term_label": "cytoplasm",
  "gene_symbol": "YWHAH",
  "gene_name": "14-3-3 protein eta",
  "gene": "UniProtKB:Q04917"
}